{
  "term_label": "neuron projection development",
  "term_id": "GO:0031175",
  "gene": "UniProtKB:Q00536",
  "gene_symbol": "CDK16",
  "gene_name": "Cyclin-dependent kinase 16"
}